protein localization to cytoplasmic microtubule plus-end [GO:1904518] (biological process) Relationships: is a type of protein localization to microtubule plus-end [GO:1904825]; is a type of protein localization to cytoplasmic microtubule [GO:1905755] References: PMID:15772152 Sources: GOC:TermGenie, GO_REF:0000087 Also known as: protein localisation in cytoplasmic microtubule plus-end, protein localisation to cytoplasmic microtubule plus-end, protein localization in cytoplasmic microtubule plus-end Definition: A process in which a protein is transported to, or maintained in, a location at a cytoplasmic microtubule plus-end.